bilirubin conjugation [GO:0006789] (biological process) Definition: The chemical reactions and pathways resulting in the formation of bilirubin monoglucuronide or bilirubin diglucuronide, water-soluble derivatives of bilirubin. Sources: DOI:10.1016/0305-0491(80)90243-6 Relationships: is a type of porphyrin-containing compound catabolic process [GO:0006787]